{
  "gene_symbol": "TMEM243",
  "gene_name": "Transmembrane protein 243",
  "gene": "UniProtKB:Q9BU79",
  "term_id": "UNKNOWN:0002",
  "term_label": "Unknown biological process"
}